{
  "gene_name": "NACHT, LRR and PYD domains-containing protein 3",
  "term_id": "GO:1901223",
  "gene_symbol": "NLRP3",
  "gene": "UniProtKB:Q96P20",
  "term_label": "negative regulation of non-canonical NF-kappaB signal transduction"
}